{
  "term_id": "GO:0000122",
  "gene_name": "Metastasis-associated protein MTA2",
  "term_label": "negative regulation of transcription by RNA polymerase II",
  "gene_symbol": "MTA2",
  "gene": "UniProtKB:O94776"
}